{
  "gene_symbol": "SLC22A18",
  "gene_name": "Solute carrier family 22 member 18",
  "gene": "UniProtKB:Q96BI1",
  "term_label": "xenobiotic detoxification by transmembrane export across the plasma membrane",
  "term_id": "GO:1990961"
}